dinoflagellate hypocone [GO:0097614] (cellular component) Definition: The part of a dinoflagellate cell below the cingulum; also referred to as the posterior portion of a dinoflagellate cell. It is separated from the epicone by the cingulum. Also known as: hypocone, hyposome, hypotheca Sources: GOC:at, Wikipedia:Dinoflagellate#Morphology, http://tolweb.org/Dinoflagellates/2445 Relationships: is a type of GO:0110165 Note: The term name refers to a taxonomic group to make the label unique with respect to similarly-named anatomical structures.